{
  "gene_symbol": "ARHGEF16",
  "term_id": "GO:0032956",
  "term_label": "regulation of actin cytoskeleton organization",
  "gene_name": "Rho guanine nucleotide exchange factor 16",
  "gene": "UniProtKB:Q5VV41"
}